{
  "term_label": "extracellular space",
  "gene_name": "Nidogen-2",
  "gene": "UniProtKB:Q14112",
  "term_id": "GO:0005615",
  "gene_symbol": "NID2"
}